fructose-1-phosphate aldolase activity [GO:0061609] (molecular function) Definition: Catalysis of the reaction: beta-D-fructose-1-phosphate = D-glyceraldehyde + dihydroxyacetone phosphate. Sources: GOC:dph, GOC:glycolysis, ISBN:0201090910, RHEA:30851 Relationships: is a type of aldehyde-lyase activity [GO:0016832]